dimethylallyl diphosphate metabolic process [GO:0050993] (biological process) Sources: GOC:ai Relationships: is a type of phospholipid metabolic process [GO:0006644] Also known as: DPP metabolic process, DPP metabolism, dimethylallyl diphosphate metabolism, dimethylallyl pyrophosphate metabolic process, dimethylallyl pyrophosphate metabolism Subtypes: GO:0050992 Definition: The chemical reactions and pathways involving dimethylallyl diphosphate.